{
  "term_id": "GO:0050660",
  "gene": "UniProtKB:Q8IWF2",
  "gene_symbol": "FOXRED2",
  "gene_name": "FAD-dependent oxidoreductase domain-containing protein 2",
  "term_label": "flavin adenine dinucleotide binding"
}